U6 snRNA binding [GO:0017070] (MF) Definition: Binding to a U6 small nuclear RNA (U6 snRNA). Sources: GOC:mah Relationships: is a type of snRNA binding [GO:0017069] Subtypes: U6 snRNA 3'-end binding [GO:0030629]